{
  "term_id": "UNKNOWN:0003",
  "gene": "UniProtKB:Q6P3W6",
  "term_label": "Unknown cellular component",
  "gene_symbol": "NBPF10",
  "gene_name": "Neuroblastoma breakpoint family member 10"
}